{
  "gene": "UniProtKB:Q8NEJ9",
  "term_id": "GO:0005730",
  "gene_symbol": "NGDN",
  "gene_name": "Neuroguidin",
  "term_label": "nucleolus"
}